striated muscle hypertrophy [GO:0014897] (biological process) Sources: GOC:mtg_muscle Subtypes: cardiac muscle hypertrophy [GO:0003300], skeletal muscle hypertrophy [GO:0014734] Definition: The enlargement or overgrowth of all or part of an organ due to an increase in size of muscle cells without cell division. In the case of striated muscle, this happens due to the additional synthesis of sarcomeric proteins and assembly of myofibrils. Relationships: is a type of GO:0014896